{
  "gene_name": "Ubiquitin domain-containing protein TINCR",
  "gene": "UniProtKB:A0A2R8Y7D0",
  "term_label": "Unknown biological process",
  "term_id": "UNKNOWN:0002",
  "gene_symbol": "TINCR"
}